cellular response to ciliary neurotrophic factor [GO:1904392] (biological process) Definition: Any process that results in a change in state or activity of a cell (in terms of movement, secretion, enzyme production, gene expression, etc.) as a result of a ciliary neurotrophic factor stimulus. References: PMID:16914133 Sources: GOC:TermGenie, GO_REF:0000071 Relationships: is a type of cellular response to nitrogen compound [GO:1901699]; is a type of response to ciliary neurotrophic factor [GO:1904391]